{
  "term_label": "Unknown biological process",
  "gene": "UniProtKB:P49223",
  "gene_name": "Kunitz-type protease inhibitor 3",
  "term_id": "UNKNOWN:0002",
  "gene_symbol": "SPINT3"
}